positive regulation of nuclear cell cycle DNA replication [GO:0010571] (biological process) Sources: GOC:mtg_cell_cycle Subtypes: positive regulation of mitotic cell cycle DNA replication [GO:1903465], positive regulation of initiation of premeiotic DNA replication [GO:1904514] Definition: Any process that activates or increases the frequency, rate or extent of the DNA-dependent DNA replication that occurs in the nucleus of eukaryotic organisms as part of the cell cycle. Also known as: positive regulation of DNA replication involved in S phase, positive regulation of DNA replication involved in S-phase, positive regulation of DNA replication during S phase Relationships: is a type of regulation of nuclear cell cycle DNA replication [GO:0033262]; is a type of positive regulation of cell cycle process [GO:0090068]; is a type of GO:2000105; positively regulates nuclear DNA replication [GO:0033260]